{
  "term_label": "Golgi apparatus",
  "gene_symbol": "YIPF3",
  "term_id": "GO:0005794",
  "gene_name": "Protein YIPF3",
  "gene": "UniProtKB:Q9GZM5"
}